{
  "gene_name": "Transcription initiation factor TFIID subunit 4B",
  "term_id": "GO:0006367",
  "gene": "UniProtKB:Q92750",
  "term_label": "transcription initiation at RNA polymerase II promoter",
  "gene_symbol": "TAF4B"
}